{
  "gene_symbol": "PEX6",
  "term_id": "GO:0005829",
  "term_label": "cytosol",
  "gene_name": "Peroxisomal ATPase PEX6",
  "gene": "UniProtKB:Q13608"
}